regulation of branching involved in mammary cord morphogenesis by fat precursor cell-epithelial cell signaling [GO:0060656] (biological process) Definition: Any process that modulates the rate, frequency, or extent of branching of the mammary gland cord as a result of a signal being created by a mammary fat precursor cell and its subsequent reception and interpretation by a mammary cord epithelial cell. Also known as: regulation of branching involved in mammary cord morphogenesis by fat precursor cell-epithelial cell signalling References: PMID:12558599 Sources: GOC:dph Relationships: is a type of cell-cell signaling [GO:0007267]; is_a regulation of branching involved in mammary gland duct morphogenesis [GO:0060762]; regulates branching involved in mammary gland cord morphogenesis [GO:0060655]